{
  "gene_symbol": "CCR7",
  "gene": "UniProtKB:P32248",
  "gene_name": "C-C chemokine receptor type 7",
  "term_label": "calcium-mediated signaling",
  "term_id": "GO:0019722"
}